{
  "term_label": "multivesicular body",
  "gene_symbol": "SFTPA2",
  "gene": "UniProtKB:Q8IWL1",
  "term_id": "GO:0005771",
  "gene_name": "Pulmonary surfactant-associated protein A2"
}